positive regulation of endocardial cushion to mesenchymal transition involved in heart valve formation [GO:2000802] (biological process) Relationships: is a type of GO:0140051; is a type of regulation of endocardial cushion to mesenchymal transition involved in heart valve formation [GO:2000800]; RO_0002213 GO:0003199 Definition: Any process that activates or increases the frequency, rate or extent of endocardial cushion to mesenchymal transition involved in heart valve formation. Also known as: positive regulation of endocardial cushion to mesenchymal transition involved in valve formation Sources: GOC:BHF